{
  "gene_symbol": "LRRC9",
  "gene_name": "Leucine-rich repeat-containing protein 9",
  "term_label": "Unknown biological process",
  "term_id": "UNKNOWN:0002",
  "gene": "UniProtKB:Q6ZRR7"
}